positive regulation of protein localization to Cajal body [GO:1904871] (biological process) Also known as: positive regulation of protein localisation in Cajal body, positive regulation of protein localisation to Cajal body, positive regulation of protein localization in Cajal body, up regulation of protein localisation in Cajal body, up regulation of protein localisation to Cajal body, up regulation of protein localization in Cajal body, up regulation of protein localization to Cajal body, up-regulation of protein localisation in Cajal body, up-regulation of protein localisation to Cajal body, up-regulation of protein localization in Cajal body, up-regulation of protein localization to Cajal body, upregulation of protein localisation in Cajal body, upregulation of protein localisation to Cajal body, upregulation of protein localization in Cajal body, upregulation of protein localization to Cajal body, activation of protein localisation in Cajal body, activation of protein localisation to Cajal body, activation of protein localization in Cajal body, activation of protein localization to Cajal body Relationships: is a type of positive regulation of protein localization to nucleus [GO:1900182]; is a type of GO:1904869; positively regulates protein localization to Cajal body [GO:1904867] Definition: Any process that activates or increases the frequency, rate or extent of protein localization to Cajal body. References: PMID:25467444 Sources: GOC:BHF, GOC:BHF_telomere, GOC:TermGenie, GOC:nc, GO_REF:0000058